{
  "term_label": "microtubule binding",
  "term_id": "GO:0008017",
  "gene_symbol": "CCDC170",
  "gene_name": "Coiled-coil domain-containing protein 170",
  "gene": "UniProtKB:Q8IYT3"
}